positive regulation of lymphangiogenesis [GO:1901492] (biological process) Definition: Any process that activates or increases the frequency, rate or extent of lymphangiogenesis. References: PMID:20133819 Sources: GOC:TermGenie, GOC:dph Also known as: positive regulation of lymph vessel formation, up regulation of lymph vessel formation, up regulation of lymphangiogenesis, up-regulation of lymph vessel formation, up-regulation of lymphangiogenesis, upregulation of lymph vessel formation, upregulation of lymphangiogenesis, activation of lymph vessel formation, activation of lymphangiogenesis Relationships: is a type of positive regulation of developmental process [GO:0051094]; is a type of regulation of lymphangiogenesis [GO:1901490]; positively regulates GO:0001946